{
  "term_id": "GO:0000981",
  "gene": "UniProtKB:Q99811",
  "term_label": "DNA-binding transcription factor activity, RNA polymerase II-specific",
  "gene_symbol": "PRRX2",
  "gene_name": "Paired mesoderm homeobox protein 2"
}